negative regulation of ferulate catabolic process [GO:1901467] (biological process) Also known as: down regulation of ferulate breakdown, down regulation of ferulate catabolic process, down regulation of ferulate catabolism, down regulation of ferulate degradation, down-regulation of ferulate breakdown, down-regulation of ferulate catabolic process, down-regulation of ferulate catabolism, down-regulation of ferulate degradation, downregulation of ferulate breakdown, downregulation of ferulate catabolic process, downregulation of ferulate catabolism, downregulation of ferulate degradation, inhibition of ferulate breakdown, inhibition of ferulate catabolism, inhibition of ferulate degradation, negative regulation of ferulate breakdown, negative regulation of ferulate catabolism, negative regulation of ferulate degradation, inhibition of ferulate catabolic process Relationships: is a type of negative regulation of catabolic process [GO:0009895]; is a type of negative regulation of small molecule metabolic process [GO:0062014]; is a type of regulation of ferulate catabolic process [GO:1901466]; negatively regulates ferulate catabolic process [GO:1901067] Sources: GOC:TermGenie, GOC:mengo_curators Definition: Any process that stops, prevents or reduces the frequency, rate or extent of ferulate catabolic process.